{
  "term_label": "G protein-coupled receptor activity",
  "gene": "UniProtKB:Q8IZF7",
  "gene_symbol": "ADGRF2P",
  "gene_name": "Adhesion G-protein coupled receptor F2",
  "term_id": "GO:0004930"
}